{
  "term_id": "GO:0005634",
  "gene_name": "Histone H2B type 1-H",
  "gene": "UniProtKB:Q93079",
  "term_label": "nucleus",
  "gene_symbol": "H2BC9"
}